{
  "gene_name": "Cysteine-rich protein 2-binding protein",
  "term_id": "GO:0004402",
  "gene": "UniProtKB:Q9H8E8",
  "gene_symbol": "KAT14",
  "term_label": "histone acetyltransferase activity"
}